{
  "gene_name": "NEDD4-like E3 ubiquitin-protein ligase WWP2",
  "gene_symbol": "WWP2",
  "gene": "UniProtKB:O00308",
  "term_id": "GO:0061630",
  "term_label": "ubiquitin protein ligase activity"
}